{
  "term_label": "G protein-coupled receptor activity",
  "term_id": "GO:0004930",
  "gene": "UniProtKB:Q9HBW9",
  "gene_name": "Adhesion G protein-coupled receptor L4",
  "gene_symbol": "ADGRL4"
}